{
  "gene": "UniProtKB:P41146",
  "gene_symbol": "OPRL1",
  "term_id": "GO:0001626",
  "term_label": "nociceptin receptor activity",
  "gene_name": "Nociceptin receptor"
}